cilium organization [GO:0044782] (biological process) Definition: A process that is carried out at the cellular level which results in the assembly, arrangement of constituent parts, or disassembly of a cilium, a specialized eukaryotic organelle that consists of a filiform extrusion of the cell surface. Each cilium is bounded by an extrusion of the cytoplasmic membrane, and contains a regular longitudinal array of microtubules, anchored basally in a centriole. Note: Note that we deem cilium and microtubule-based flagellum to be equivalent. Sources: GOC:cilia, GOC:jl Relationships: is a type of organelle organization [GO:0006996]; is_a plasma membrane bounded cell projection organization [GO:0120036] Also known as: microtubule-based flagellum organization Subtypes: ciliary basal body organization [GO:0032053], cilium assembly [GO:0060271], cilium disassembly [GO:0061523]